S-adenosylmethionine metabolic process [GO:0046500] (biological process) Relationships: is a type of sulfur compound metabolic process [GO:0006790] Subtypes: S-adenosylmethionine biosynthetic process [GO:0006556], GO:0033353, S-adenosylmethionine catabolic process [GO:0050843] Sources: GOC:go_curators, ISBN:0198506732 Also known as: S-adenosyl methionine metabolic process, S-adenosyl methionine metabolism, S-adenosylmethionine metabolism, SAM metabolic process Definition: The chemical reactions and pathways involving S-adenosylmethionine, S-(5'-adenosyl)-L-methionine, an important intermediate in one-carbon metabolism.